positive regulation of response to gamma radiation [GO:2001230] (biological process) Also known as: positive regulation of response to gamma ray, positive regulation of response to gamma-ray photon Sources: GOC:obol Relationships: is a type of positive regulation of response to stimulus [GO:0048584]; is a type of regulation of response to gamma radiation [GO:2001228]; positively regulates response to gamma radiation [GO:0010332] Subtypes: GO:1905845 Definition: Any process that activates or increases the frequency, rate or extent of response to gamma radiation.